{
  "gene_symbol": "PITX2",
  "term_label": "nucleus",
  "gene": "UniProtKB:Q99697",
  "gene_name": "Pituitary homeobox 2",
  "term_id": "GO:0005634"
}